{
  "term_id": "GO:0004052",
  "gene_symbol": "ALOX12",
  "gene": "UniProtKB:P18054",
  "gene_name": "Polyunsaturated fatty acid lipoxygenase ALOX12",
  "term_label": "arachidonate 12(S)-lipoxygenase activity"
}